ventral disc microtubule array [GO:0097593] (cellular component) Relationships: is a type of GO:0110165; is part of ventral disc [GO:0097597]; has part microtubule [GO:0005874] Sources: GOC:giardia Also known as: spiral microtubule array, ventral disc spiral microtubule array, ventral disk microtubule array Definition: A part of the ventral disc of Giardia species (trophozoite stage) consisting of a spiral array of microtubules linked to the ventral membrane. These microtubules form the base of the ventral disc dorsal microribbons that extend nearly perpendicular from the membrane. Note: Due to the asymmetric nature of the Giardia trophozoite, this term is defined spatially as the trophozoite is viewed from the dorsal side, with the two nuclei dorsal to the ventral disc, and the ventral disc toward the anterior.